SCF complex assembly [GO:0010265] (biological process) Sources: GOC:pz Definition: The aggregation, arrangement and bonding together of a set of components to form the SKP1-Cullin/Cdc53-F-box protein ubiquitin ligase (SCF) complex. Relationships: is a type of GO:0065003